{
  "term_label": "phospholipid metabolic process",
  "gene_name": "Phospholipid phosphatase-related protein type 1",
  "gene": "UniProtKB:Q8TBJ4",
  "gene_symbol": "PLPPR1",
  "term_id": "GO:0006644"
}